{
  "term_id": "GO:0005739",
  "gene": "UniProtKB:Q6ZS86",
  "term_label": "mitochondrion",
  "gene_name": "Putative glycerol kinase 5",
  "gene_symbol": "GK5"
}